beta-glucoside catabolic process [GO:1901805] (biological process) Subtypes: GO:1901829, ergosteryl 3-beta-D-glucoside catabolic process [GO:1904462] Definition: The chemical reactions and pathways resulting in the breakdown of beta-glucoside. References: PMID:15205427, PMID:16390337, PMID:8990303 Sources: GOC:TermGenie, GOC:yaf, Unipathway:UPA00237 Also known as: beta-glucoside breakdown, beta-glucoside catabolism, beta-glucoside degradation Relationships: is a type of glycoside catabolic process [GO:0016139]